{
  "gene_symbol": "RUNX3",
  "gene_name": "Runt-related transcription factor 3",
  "term_label": "RNA polymerase II cis-regulatory region sequence-specific DNA binding",
  "term_id": "GO:0000978",
  "gene": "UniProtKB:Q13761"
}